{
  "gene_symbol": "SGK3",
  "gene_name": "Serine_threonine-protein kinase Sgk3",
  "gene": "UniProtKB:Q96BR1",
  "term_id": "GO:0035556",
  "term_label": "intracellular signal transduction"
}